{
  "gene_symbol": "RORB",
  "gene_name": "Nuclear receptor ROR-beta",
  "term_id": "GO:0006357",
  "term_label": "regulation of transcription by RNA polymerase II",
  "gene": "UniProtKB:Q92753"
}